{
  "term_label": "Unknown molecular function",
  "gene": "UniProtKB:Q9H609",
  "term_id": "UNKNOWN:0001",
  "gene_symbol": "ZNF576",
  "gene_name": "Zinc finger protein 576"
}